{
  "gene": "UniProtKB:Q99933",
  "term_id": "GO:0051087",
  "term_label": "protein-folding chaperone binding",
  "gene_name": "BAG family molecular chaperone regulator 1",
  "gene_symbol": "BAG1"
}